{
  "term_id": "GO:0030424",
  "term_label": "axon",
  "gene_symbol": "HCN1",
  "gene": "UniProtKB:O60741",
  "gene_name": "Potassium_sodium hyperpolarization-activated cyclic nucleotide-gated channel 1"
}